{
  "gene_symbol": "PPP1R27",
  "gene_name": "Protein phosphatase 1 regulatory subunit 27",
  "term_id": "GO:0019902",
  "term_label": "phosphatase binding",
  "gene": "UniProtKB:Q86WC6"
}